{
  "term_id": "GO:1990410",
  "gene_symbol": "ADM",
  "gene": "UniProtKB:P35318",
  "gene_name": "Pro-adrenomedullin",
  "term_label": "adrenomedullin receptor signaling pathway"
}